eclosion hormone activity [GO:0008031] (molecular function) Definition: The action characteristic of eclosion hormone, a peptide hormone that, upon receptor binding, triggers the death of certain muscles and neurons during insect metamorphosis. Relationships: is a type of neuropeptide hormone activity [GO:0005184] Sources: GOC:mah, ISBN:0198506732